H3 histone acetyltransferase complex [GO:0070775] (cellular component) Definition: A multisubunit complex that catalyzes the acetylation of histone H3. Sources: GOC:mah Also known as: H3 HAT complex Relationships: is a type of histone acetyltransferase complex [GO:0000123] Subtypes: NuA3 histone acetyltransferase complex [GO:0033100], histone H3-K14 acetyltransferase complex [GO:0036409], MOZ/MORF histone acetyltransferase complex [GO:0070776], Hpa2 acetyltransferase complex [GO:1990331]